{
  "gene_name": "Lymphotactin",
  "term_id": "GO:0048020",
  "gene": "UniProtKB:P47992",
  "gene_symbol": "XCL1",
  "term_label": "CCR chemokine receptor binding"
}